ethanol dehydrogenase (NAD+) activity [GO:0120542] (molecular function) Relationships: is a type of alcohol dehydrogenase (NAD+) activity [GO:0004022] Definition: Catalysis of the reaction: ethanol + NAD+ = acetaldehyde + NADH + H+. Sources: RHEA:25290